gamma-glutamylcyclotransferase activity [GO:0003839] (molecular function) Relationships: is a type of amidine-lyase activity [GO:0016842] Definition: Catalysis of the reaction: (5-L-glutamyl)-L-amino acid = 5-oxoproline + L-amino acid. Also known as: (5-L-glutamyl)-L-amino-acid 5-glutamyltransferase (cyclizing), L-glutamic cyclase activity, gamma-L-glutamylcyclotransferase activity, gamma-glutamyl-amino acid cyclotransferase activity References: PMID:18515354